{
  "gene_symbol": "PLEKHA8",
  "term_label": "ceramide 1-phosphate transfer activity",
  "gene": "UniProtKB:Q96JA3",
  "term_id": "GO:1902388",
  "gene_name": "Pleckstrin homology domain-containing family A member 8"
}